{
  "term_label": "Unknown cellular component",
  "gene_name": "Di-N-acetylchitobiase",
  "gene_symbol": "CTBS",
  "term_id": "UNKNOWN:0003",
  "gene": "UniProtKB:Q01459"
}